regulation of caveolin-mediated endocytosis [GO:2001286] (biological process) Definition: Any process that modulates the frequency, rate or extent of caveolin-mediated endocytosis. Also known as: regulation of caveolae-dependent endocytosis, regulation of caveolae-mediated endocytosis, regulation of caveolin-dependent endocytosis Subtypes: negative regulation of caveolin-mediated endocytosis [GO:2001287], positive regulation of caveolin-mediated endocytosis [GO:2001288] Relationships: is a type of regulation of endocytosis [GO:0030100]; regulates caveolin-mediated endocytosis [GO:0072584] Sources: GOC:obol